{
  "gene": "UniProtKB:Q8NFJ9",
  "gene_symbol": "BBS1",
  "term_id": "GO:1905515",
  "gene_name": "Bardet-Biedl syndrome 1 protein",
  "term_label": "non-motile cilium assembly"
}